regulation of endothelial cell proliferation [GO:0001936] (biological process) Definition: Any process that modulates the frequency, rate, or extent of endothelial cell proliferation. Relationships: is a type of regulation of epithelial cell proliferation [GO:0050678]; regulates GO:0001935 Subtypes: negative regulation of endothelial cell proliferation [GO:0001937], positive regulation of endothelial cell proliferation [GO:0001938], regulation of blood vessel endothelial cell proliferation involved in sprouting angiogenesis [GO:1903587], regulation of vascular endothelial cell proliferation [GO:1905562] Sources: GOC:add